{
  "gene_name": "Sphingosine 1-phosphate receptor 3",
  "term_id": "GO:0007189",
  "gene": "UniProtKB:Q99500",
  "gene_symbol": "S1PR3",
  "term_label": "adenylate cyclase-activating G protein-coupled receptor signaling pathway"
}